Y-shaped link [GO:0097537] (cellular component) Also known as: Y-link, Y-link structure, Y-shaped assemblage, Y-shaped fiber, Y-shaped fibre, Y-shaped linker, membrane-microtubule complex Relationships: is a type of protein-containing complex [GO:0032991]; is part of GO:0035869 Definition: A Y-shaped protein complex in the ciliary transition zone that connects the cilium axoneme to the ciliary necklace. Both protein sorting and protein gating occur at this point in the cilium allowing some, but not all proteins to enter the cilium. References: PMID:22653444, PMID:4554367 Sources: GOC:cilia